L-tyrosine binding [GO:0072545] (molecular function) Sources: GOC:mah Relationships: is_a amino acid binding [GO:0016597]; is a type of carboxylic acid binding [GO:0031406]; is a type of cation binding [GO:0043169] Also known as: tyrosine binding, L-Tyr binding Definition: Binding to L-tyrosine, 2-amino-3-(4-hydroxyphenyl)propanoic acid.